lung proximal/distal axis specification [GO:0061115] (biological process) Relationships: is a type of proximal/distal axis specification [GO:0009946]; is a type of lung pattern specification process [GO:0060432] Sources: GOC:dph Definition: The establishment, maintenance and elaboration of the proximal/distal axis of the lung. The proximal/distal axis of the lung is defined by a line that runs from the trachea to the alveoli.